adult chitin-based cuticle pattern formation [GO:0035018] (biological process) Relationships: is a type of cuticle pattern formation [GO:0035017]; is part of adult chitin-based cuticle development [GO:0008365] Also known as: adult cuticle pattern formation Sources: GOC:bf, GOC:mtg_sensu Definition: The process that gives rise to the patterns of cell differentiation that will arise in the chitin-based adult cuticle. An example of this process is adult chitin-based cuticle pattern formation in Drosophila melanogaster.